{
  "gene_name": "Semaphorin-7A",
  "term_id": "GO:0050919",
  "gene_symbol": "SEMA7A",
  "term_label": "negative chemotaxis",
  "gene": "UniProtKB:O75326"
}